{
  "gene_name": "Translocating chain-associated membrane protein 1-like 1",
  "term_id": "GO:0045048",
  "term_label": "protein insertion into ER membrane",
  "gene": "UniProtKB:Q8N609",
  "gene_symbol": "TRAM1L1"
}